arabinose metabolic process [GO:0019566] (BP) Relationships: is a type of pentose metabolic process [GO:0019321] Also known as: arabinose metabolism Subtypes: GO:0019567, GO:0019568, L-arabinose metabolic process [GO:0046373] Sources: ISBN:0198506732 Definition: The chemical reactions and pathways involving arabinose, arabino-pentose. L-Arabinose occurs both free, for example in the heartwood of many conifers, and in the combined state, as a constituent of plant hemicelluloses, bacterial polysaccharides etc. D-arabinose is a constituent of arabinonucleosides.